periodic partitioning by pair rule gene [GO:0007366] (biological process) Relationships: is a type of periodic partitioning [GO:0007365]; is a type of anterior/posterior pattern specification [GO:0009952] Definition: Allocation of cells to parasegments in the embryo, through the action of overlapping series of pair rule gene activities. Sources: ISBN:0632030488, ISBN:0879694238, http://fly.ebi.ac.uk/allied-data/lk/interactive-fly/aimain/1aahome.htm